{
  "gene_symbol": "PIWIL1",
  "term_id": "GO:0005634",
  "gene_name": "Piwi-like protein 1",
  "term_label": "nucleus",
  "gene": "UniProtKB:Q96J94"
}